{
  "term_label": "mismatch repair complex",
  "gene_symbol": "MLH3",
  "gene_name": "DNA mismatch repair protein Mlh3",
  "gene": "UniProtKB:Q9UHC1",
  "term_id": "GO:0032300"
}